{
  "gene": "UniProtKB:P0CAP1",
  "term_label": "Unknown molecular function",
  "gene_symbol": "MYZAP",
  "term_id": "UNKNOWN:0001",
  "gene_name": "Myocardial zonula adherens protein"
}